{
  "gene": "UniProtKB:Q04771",
  "gene_name": "Activin receptor type-1",
  "term_id": "GO:0005025",
  "gene_symbol": "ACVR1",
  "term_label": "transforming growth factor beta receptor activity, type I"
}